{
  "gene_symbol": "MFSD12",
  "gene": "UniProtKB:Q6NUT3",
  "gene_name": "Major facilitator superfamily domain-containing protein 12",
  "term_label": "pigment metabolic process involved in pigmentation",
  "term_id": "GO:0043474"
}